{
  "term_label": "DNA binding",
  "gene": "UniProtKB:Q16526",
  "term_id": "GO:0003677",
  "gene_name": "Cryptochrome-1",
  "gene_symbol": "CRY1"
}